interferon regulatory factor 5 complex [GO:0097073] (CC) References: PMID:12138184, PMID:16751392 Sources: GOC:cna Relationships: is a type of interferon regulatory factor complex [GO:0097071] Also known as: IRF5:IRF5 complex Definition: An interferon regulatory factor complex that consists of a homodimer of interferon regulatory factor 5.